{
  "gene": "UniProtKB:Q8N6D5",
  "term_id": "UNKNOWN:0003",
  "gene_name": "Ankyrin repeat domain-containing protein 29",
  "gene_symbol": "ANKRD29",
  "term_label": "Unknown cellular component"
}